{
  "gene_symbol": "SLC39A11",
  "term_label": "membrane",
  "gene_name": "Zinc transporter ZIP11",
  "term_id": "GO:0016020",
  "gene": "UniProtKB:Q8N1S5"
}